negative regulation of adherens junction organization [GO:1903392] (biological process) References: PMID:21724833 Sources: GOC:TermGenie, GOC:als, GO_REF:0000058 Also known as: down regulation of adherens junction assembly and maintenance, down regulation of adherens junction organisation, down regulation of adherens junction organization, down-regulation of adherens junction assembly and maintenance, down-regulation of adherens junction organisation, down-regulation of adherens junction organization, downregulation of adherens junction assembly and maintenance, downregulation of adherens junction organisation, downregulation of adherens junction organization, negative regulation of adherens junction assembly and maintenance, negative regulation of adherens junction organisation, inhibition of adherens junction assembly and maintenance, inhibition of adherens junction organisation, inhibition of adherens junction organization Relationships: is_a negative regulation of cellular component organization [GO:0051129]; is a type of GO:1903391; negatively regulates GO:0034332 Definition: Any process that stops, prevents or reduces the frequency, rate or extent of adherens junction organization.